sulfate binding [GO:0043199] (MF) Sources: GOC:mlg Relationships: is a type of anion binding [GO:0043168]; is a type of sulfur compound binding [GO:1901681] Definition: Binding to sulfate, SO4(2-), a negatively charged small molecule.